{
  "gene_symbol": "CASP9",
  "term_label": "intrinsic apoptotic signaling pathway in response to DNA damage",
  "gene_name": "Caspase-9",
  "gene": "UniProtKB:P55211",
  "term_id": "GO:0008630"
}